spindle assembly involved in female meiosis II [GO:0007058] (biological process) Relationships: is a type of spindle assembly involved in female meiosis [GO:0007056]; is part of female meiosis II [GO:0007147] Sources: GOC:mah Definition: The aggregation, arrangement and bonding together of a set of components to form the spindle during meiosis II of a meiotic cell cycle in females. An example of this is found in Drosophila melanogaster. Also known as: female meiosis II spindle assembly